{
  "term_id": "UNKNOWN:0002",
  "term_label": "Unknown biological process",
  "gene_name": "Cubilin",
  "gene_symbol": "CUBN",
  "gene": "UniProtKB:O60494"
}